regulation of lipid metabolic process [GO:0019216] (biological process) Subtypes: regulation of fatty acid metabolic process [GO:0019217], regulation of steroid metabolic process [GO:0019218], regulation of isoprenoid metabolic process [GO:0019747], GO:0045833, positive regulation of lipid metabolic process [GO:0045834], regulation of lipid biosynthetic process [GO:0046890], regulation of lipid catabolic process [GO:0050994], regulation of lipoprotein lipid oxidation [GO:0060587], GO:0090207, regulation of phospholipid metabolic process [GO:1903725], GO:1905038 Relationships: is a type of regulation of primary metabolic process [GO:0080090]; regulates lipid metabolic process [GO:0006629] Definition: Any process that modulates the frequency, rate or extent of the chemical reactions and pathways involving lipids. Also known as: regulation of lipid metabolism Sources: GOC:go_curators